{
  "gene": "UniProtKB:Q17RH7",
  "term_label": "Unknown cellular component",
  "gene_name": "Tetra-peptide repeat homeobox-like protein",
  "gene_symbol": "TPRXL",
  "term_id": "UNKNOWN:0003"
}